cycloheximide transport [GO:0015901] (biological process) Relationships: is a type of organic hydroxy compound transport [GO:0015850]; is a type of GO:0042886 Definition: The directed movement of cycloheximide into, out of or within a cell, or between cells, by means of some agent such as a transporter or pore. Cycloheximide is an antibiotic produced by Streptomyces which interferes with protein synthesis in eukaryotes. Sources: ISBN:0198506732